primary growth [GO:0080189] (BP) Definition: Growth of a plant structure from the time of its initiation by an apical meristem until its expansion is completed. Relationships: is a type of multicellular organismal process [GO:0032501]; is a type of growth [GO:0040007] Note: Has its inception in the apical meristems (PO:0020144) and continues in their derivative meristems - protoderm (PO:0006210) and procambium (PO:0025275) - even in older tissues. Primary and secondary growth can occur simultaneously in the same organism. Sources: ISBN:0471245208